{
  "gene_name": "Humanin-like 13",
  "gene_symbol": "MTRNR2L13",
  "gene": "UniProtKB:S4R3P1",
  "term_id": "GO:1900118",
  "term_label": "negative regulation of execution phase of apoptosis"
}